{
  "term_label": "vesicle-mediated transport",
  "gene": "UniProtKB:P21579",
  "term_id": "GO:0016192",
  "gene_name": "Synaptotagmin-1",
  "gene_symbol": "SYT1"
}